{
  "gene_name": "Transcription elongation factor SPT4",
  "term_id": "GO:0032044",
  "gene": "UniProtKB:P63272",
  "gene_symbol": "SUPT4H1",
  "term_label": "DSIF complex"
}